{
  "term_id": "GO:0032870",
  "gene_symbol": "QRFPR",
  "gene": "UniProtKB:Q96P65",
  "term_label": "cellular response to hormone stimulus",
  "gene_name": "Pyroglutamylated RF-amide peptide receptor"
}